{
  "gene": "UniProtKB:Q9Y3V2",
  "term_id": "UNKNOWN:0003",
  "gene_name": "RWD domain-containing protein 3",
  "gene_symbol": "RWDD3",
  "term_label": "Unknown cellular component"
}